{
  "term_label": "extracellular space",
  "gene_name": "Granulocyte-macrophage colony-stimulating factor",
  "gene_symbol": "CSF2",
  "term_id": "GO:0005615",
  "gene": "UniProtKB:P04141"
}